{
  "gene": "UniProtKB:Q86TJ2",
  "gene_symbol": "TADA2B",
  "term_label": "transcription coactivator activity",
  "term_id": "GO:0003713",
  "gene_name": "Transcriptional adapter 2-beta"
}